{
  "term_label": "lysosome",
  "gene_name": "Sialidase-2",
  "gene": "UniProtKB:Q9Y3R4",
  "term_id": "GO:0005764",
  "gene_symbol": "NEU2"
}